{
  "gene_name": "C-C chemokine receptor type 2",
  "gene_symbol": "CCR2",
  "gene": "UniProtKB:P41597",
  "term_id": "GO:0016493",
  "term_label": "C-C chemokine receptor activity"
}